{
  "gene_symbol": "TTBK2",
  "gene_name": "Tau-tubulin kinase 2",
  "gene": "UniProtKB:Q6IQ55",
  "term_label": "signal transduction",
  "term_id": "GO:0007165"
}